{
  "term_label": "paracellular transport",
  "term_id": "GO:0160184",
  "gene_name": "Claudin-16",
  "gene_symbol": "CLDN16",
  "gene": "UniProtKB:Q9Y5I7"
}